{
  "gene_symbol": "CD68",
  "term_id": "GO:0072594",
  "gene": "UniProtKB:P34810",
  "gene_name": "Macrosialin",
  "term_label": "establishment of protein localization to organelle"
}